{
  "term_label": "Unknown molecular function",
  "gene_name": "MAM domain-containing glycosylphosphatidylinositol anchor protein 1",
  "term_id": "UNKNOWN:0001",
  "gene": "UniProtKB:Q8NFP4",
  "gene_symbol": "MDGA1"
}